{
  "gene_symbol": "MMP23B",
  "gene": "UniProtKB:O75900",
  "term_id": "GO:0005615",
  "term_label": "extracellular space",
  "gene_name": "Matrix metalloproteinase-23"
}